{
  "term_id": "GO:0000146",
  "gene": "UniProtKB:P12882",
  "gene_symbol": "MYH1",
  "gene_name": "Myosin-1",
  "term_label": "microfilament motor activity"
}